{
  "gene_name": "DAN domain family member 5",
  "term_id": "GO:0061371",
  "gene_symbol": "DAND5",
  "gene": "UniProtKB:Q8N907",
  "term_label": "determination of heart left/right asymmetry"
}